{
  "term_id": "GO:1903577",
  "gene_symbol": "CASTOR1",
  "term_label": "cellular response to L-arginine",
  "gene_name": "Cytosolic arginine sensor for mTORC1 subunit 1",
  "gene": "UniProtKB:Q8WTX7"
}